potassium channel activity [GO:0005267] (molecular function) Definition: Enables the energy-independent facilitated diffusion of a potassium ion through a transmembrane aqueous pore or channel. Relationships: is a type of monoatomic cation channel activity [GO:0005261]; is a type of potassium ion transmembrane transporter activity [GO:0015079] Sources: GOC:BHF, GOC:mtg_transport, GOC:pr, ISBN:0815340729 Subtypes: GO:0005228, voltage-gated potassium channel activity [GO:0005249], calcium-activated potassium channel activity [GO:0015269], kainate selective glutamate receptor activity [GO:0015277], potassium ion leak channel activity [GO:0022841], mitochondrial ATP-gated potassium channel activity [GO:0062156], GO:0070089, mechanosensitive potassium channel activity [GO:0098782], GO:0099101 Regulation: regulated by potassium channel regulator activity [GO:0015459]; negatively regulated by GO:0019870; positively regulated by potassium channel activator activity [GO:0099104]